{
  "gene_name": "Tubulin-specific chaperone cofactor E-like protein",
  "gene_symbol": "TBCEL",
  "term_id": "GO:0007021",
  "term_label": "tubulin complex assembly",
  "gene": "UniProtKB:Q5QJ74"
}